{
  "gene": "UniProtKB:Q13075",
  "gene_name": "Baculoviral IAP repeat-containing protein 1",
  "term_id": "GO:0004869",
  "gene_symbol": "NAIP",
  "term_label": "cysteine-type endopeptidase inhibitor activity"
}